{
  "gene_symbol": "ZFYVE1",
  "gene": "UniProtKB:Q9HBF4",
  "gene_name": "Zinc finger FYVE domain-containing protein 1",
  "term_id": "GO:0005811",
  "term_label": "lipid droplet"
}